left posteriolateral basal body [GO:1902673] (cellular component) Note: Note that we deem cilium and microtubule-based flagellum to be equivalent. Also note that, due to the asymmetric nature of the Giardia trophozoite, this term is defined spatially as the trophozoite is viewed from the dorsal side, with the two nuclei dorsal to the ventral disc, and the ventral disc toward the anterior. References: PMID:16607022, PMID:5961344 Sources: GOC:TermGenie, GOC:giardia, GO_REF:0000064, ISBN:9780124260207 Relationships: is a type of GO:0036064; is part of left posteriolateral flagellum [GO:0097556] Definition: Any ciliary basal body that is part of a left posteriolateral flagellum found in Giardia species (trophozoite stage). Also known as: cilial basal body of left posteriolateral cilium, cilial basal body of left posteriolateral flagellum, cilial basal body of left posterolateral cilium, cilial basal body of left posterolateral flagellum, ciliary basal body of left posteriolateral cilium, ciliary basal body of left posteriolateral flagellum, ciliary basal body of left posterolateral cilium, ciliary basal body of left posterolateral flagellum, cilium basal body of left posteriolateral cilium, cilium basal body of left posteriolateral flagellum, cilium basal body of left posterolateral cilium, cilium basal body of left posterolateral flagellum, left posteriolateral flagellum ciliary basal body, microtubule basal body of left posteriolateral cilium, microtubule basal body of left posteriolateral flagellum, microtubule basal body of left posterolateral cilium, microtubule basal body of left posterolateral flagellum